{
  "term_label": "animal organ morphogenesis",
  "term_id": "GO:0009887",
  "gene": "UniProtKB:Q9BYU1",
  "gene_symbol": "PBX4",
  "gene_name": "Pre-B-cell leukemia transcription factor 4"
}